{
  "gene_symbol": "NUP50",
  "term_id": "GO:0006606",
  "term_label": "protein import into nucleus",
  "gene": "UniProtKB:Q9UKX7",
  "gene_name": "Nuclear pore complex protein Nup50"
}